tight junction [GO:0070160] (CC) Definition: A cell-cell junction that seals cells together in an epithelium in a way that prevents even small molecules from leaking from one side of the sheet to the other. Sources: ISBN:0815332181 Also known as: occluding cell junction, occluding junction Relationships: is a type of cell-cell junction [GO:0005911] Subtypes: GO:0005918, GO:0005923, tricellular tight junction [GO:0061689]